{
  "gene_name": "Proteasome subunit beta type-1",
  "gene_symbol": "PSMB1",
  "term_label": "nucleus",
  "gene": "UniProtKB:P20618",
  "term_id": "GO:0005634"
}